{
  "term_label": "zinc ion binding",
  "gene_name": "Alcohol dehydrogenase 6",
  "gene_symbol": "ADH6",
  "term_id": "GO:0008270",
  "gene": "UniProtKB:P28332"
}